replacement ossification [GO:0036075] (biological process) Sources: GO_REF:0000034 Also known as: indirect ossification Subtypes: GO:0001958 Relationships: is a type of GO:0001503 Definition: Ossification that requires the replacement of a preexisting tissue prior to bone tissue formation.